radial spoke 3 [GO:0120335] (cellular component) Definition: Radial spoke 3 (RS3), when present, is the most distal of each group of radial spokes, whether grouped as triplets or doublets. RS3 has significantly different morphology and protein composition than RS1 and RS2 and also extends at a slant from the microtubule doublet, rather than perpendicularly like RS1 and RS2. In some organisms (e.g. Chlamydomonas and Sarcophaga bullata), RS3 is represented only as a stump attached to the A-microtubule lacking the rest of the stalk structure and entirely lacking the head structure. Relationships: is a type of radial spoke [GO:0001534] References: PMID:22754630, PMID:25694453, PMID:9450971 Sources: GOC:krc, ISBN:0124325653 Also known as: RS3